{
  "gene": "UniProtKB:Q9ULH7",
  "gene_symbol": "MRTFB",
  "gene_name": "Myocardin-related transcription factor B",
  "term_id": "GO:0003713",
  "term_label": "transcription coactivator activity"
}